{
  "term_id": "GO:0031012",
  "gene_symbol": "FBLN2",
  "gene_name": "Fibulin-2",
  "term_label": "extracellular matrix",
  "gene": "UniProtKB:P98095"
}